{
  "gene": "UniProtKB:Q9H6U8",
  "gene_name": "Alpha-1,2-mannosyltransferase ALG9",
  "term_id": "GO:0000026",
  "term_label": "alpha-1,2-mannosyltransferase activity",
  "gene_symbol": "ALG9"
}